{
  "gene_symbol": "HSPA1A",
  "term_id": "GO:0005886",
  "gene": "UniProtKB:P0DMV8",
  "gene_name": "Heat shock 70 kDa protein 1A",
  "term_label": "plasma membrane"
}